{
  "gene": "UniProtKB:Q7RTS1",
  "term_label": "positive regulation of transcription by RNA polymerase II",
  "gene_name": "Class A basic helix-loop-helix protein 15",
  "term_id": "GO:0045944",
  "gene_symbol": "BHLHA15"
}